{
  "gene": "UniProtKB:Q14602",
  "term_id": "UNKNOWN:0001",
  "term_label": "Unknown molecular function",
  "gene_symbol": "ID2B",
  "gene_name": "Putative DNA-binding protein inhibitor ID-2B"
}